{
  "term_id": "GO:0000981",
  "term_label": "DNA-binding transcription factor activity, RNA polymerase II-specific",
  "gene_name": "DNA-binding protein RFX2",
  "gene": "UniProtKB:P48378",
  "gene_symbol": "RFX2"
}